BLOC-1 complex [GO:0031083] (cellular component) Definition: A protein complex required for the biogenesis of specialized organelles of the endosomal-lysosomal system, such as melanosomes and platelet dense granules. Many of the protein subunits are conserved between mouse and human; the mouse complex contains the Pallidin, Muted, Cappuccino, Dysbindin, Snapin, BLOS1, BLOS2, AND BLOS3 proteins. Relationships: is a type of BLOC complex [GO:0031082] References: PMID:15102850